transcription elongation factor complex [GO:0008023] (cellular component) Sources: GOC:jl Relationships: is a type of GO:0140513; is part of nucleoplasm [GO:0005654] Subtypes: nucleoplasmic THO complex [GO:0000446], cyclin/CDK positive transcription elongation factor complex [GO:0008024], Cdc73/Paf1 complex [GO:0016593], NELF complex [GO:0032021], DSIF complex [GO:0032044], super elongation complex [GO:0032783], FACT complex [GO:0035101], elongin complex [GO:0070449] Definition: Any protein complex that interacts with RNA polymerase II to increase (positive transcription elongation factor) or reduce (negative transcription elongation factor) the rate of transcription elongation.